{
  "term_id": "GO:0031110",
  "term_label": "regulation of microtubule polymerization or depolymerization",
  "gene_symbol": "STMN2",
  "gene": "UniProtKB:Q93045",
  "gene_name": "Stathmin-2"
}